blasticidin S biosynthetic process [GO:1905266] (biological process) Definition: The chemical reactions and pathways resulting in the formation of blasticidin S. References: PMID:23874663 Sources: GOC:TermGenie, GOC:pr, GO_REF:0000068, Wikipedia:Blasticidin_S Also known as: blasticidin S anabolism, blasticidin S biosynthesis, blasticidin S formation, blasticidin S synthesis Relationships: is a type of GO:0046134